{
  "gene_name": "Signal transducer and activator of transcription 5B",
  "gene_symbol": "STAT5B",
  "term_label": "regulation of cell population proliferation",
  "term_id": "GO:0042127",
  "gene": "UniProtKB:P51692"
}